regulation of animal organ formation [GO:0003156] (biological process) Subtypes: organ induction [GO:0001759], GO:0048504, GO:0060685, regulation of heart induction [GO:0090381] Definition: Any process that modulates the rate, frequency or extent of animal organ formation. Organ formation is the process pertaining to the initial formation of an organ from unspecified parts. The process begins with the specific processes that contribute to the appearance of the discrete structure, such as inductive events, and ends when the structural rudiment of the organ is recognizable, such as a condensation of mesenchymal cells into the organ rudiment. Relationships: is a type of regulation of animal organ morphogenesis [GO:2000027]; regulates animal organ formation [GO:0048645] Sources: GOC:dph, GOC:mtg_heart, GOC:tb